{
  "gene": "UniProtKB:P60606",
  "gene_name": "Cortexin-1",
  "term_label": "Unknown biological process",
  "gene_symbol": "CTXN1",
  "term_id": "UNKNOWN:0002"
}